{
  "gene_symbol": "MEGF11",
  "term_label": "extracellular space",
  "term_id": "GO:0005615",
  "gene_name": "Multiple epidermal growth factor-like domains protein 11",
  "gene": "UniProtKB:A6BM72"
}